{
  "gene_symbol": "OLFM4",
  "gene": "UniProtKB:Q6UX06",
  "gene_name": "Olfactomedin-4",
  "term_id": "GO:0005615",
  "term_label": "extracellular space"
}